U2 snRNA adenosine m6 methyltransferase activity [GO:0106348] (molecular function) References: PMID:32637152 Relationships: is a type of snRNA methyltransferase activity [GO:0106346] Definition: Catalysis of the reaction: a adenosine in U2 snRNA + S-adenosyl-L-methionine = an N6-methyl-adenosine in U2 snRNA + S-adenosyl-L-homocysteine + H+.